{
  "gene_symbol": "NKX1-1",
  "gene": "UniProtKB:Q15270",
  "gene_name": "NK1 transcription factor-related protein 1",
  "term_id": "GO:0030154",
  "term_label": "cell differentiation"
}